negative regulation of cholesterol metabolic process [GO:0090206] (biological process) Definition: Any process that decreases the rate, frequency, or extent of cholesterol metabolism, the chemical reactions and pathways involving cholesterol, cholest-5-en-3 beta-ol, the principal sterol of vertebrates and the precursor of many steroids, including bile acids and steroid hormones. Sources: GOC:dph, GOC:sl, GOC:tb Relationships: is a type of GO:0045939; is a type of negative regulation of small molecule metabolic process [GO:0062014]; is a type of GO:0090181; negatively regulates cholesterol metabolic process [GO:0008203] Subtypes: negative regulation of cholesterol biosynthetic process [GO:0045541]